ascospore-type prospore nucleus [GO:1905754] (cellular component) Relationships: is a type of GO:0005634; is part of ascospore-type prospore [GO:0042764] References: PMID:26942678 Sources: GOC:TermGenie, GO_REF:0000064 Definition: Any nucleus that is part of a ascospore-type prospore. Also known as: cell nucleus of ascospore-type prospore, nucleus of ascospore-type prospore